{
  "gene_name": "Protocadherin beta-5",
  "term_label": "cell adhesion molecule binding",
  "gene_symbol": "PCDHB5",
  "term_id": "GO:0050839",
  "gene": "UniProtKB:Q9Y5E4"
}